{
  "term_id": "UNKNOWN:0003",
  "gene": "UniProtKB:O60303",
  "term_label": "Unknown cellular component",
  "gene_name": "Katanin-interacting protein",
  "gene_symbol": "KATNIP"
}